{
  "term_id": "GO:0000103",
  "gene_name": "Bifunctional 3'-phosphoadenosine 5'-phosphosulfate synthase 2",
  "gene": "UniProtKB:O95340",
  "gene_symbol": "PAPSS2",
  "term_label": "sulfate assimilation"
}